{
  "gene_name": "Zinc finger C3HC-type protein 1",
  "term_label": "Unknown biological process",
  "gene": "UniProtKB:Q86WB0",
  "gene_symbol": "ZC3HC1",
  "term_id": "UNKNOWN:0002"
}